{
  "gene": "UniProtKB:Q86T03",
  "gene_symbol": "PIP4P1",
  "gene_name": "Type 1 phosphatidylinositol 4,5-bisphosphate 4-phosphatase",
  "term_id": "GO:0034597",
  "term_label": "phosphatidylinositol-4,5-bisphosphate 4-phosphatase activity"
}